ferric-enterobactin import into cell [GO:0015685] (biological process) References: PMID:23192658 Sources: GOC:pg Relationships: is a type of organic anion transport [GO:0015711]; is a type of GO:0033214 Definition: A process in which ferric-enterobactin, the iron-bound form of the siderophore enterobactin, is transported into the cell by specific cell surface receptors. Also known as: ferric-enterobactin transport